selenotransferase activity [GO:0016785] (molecular function) Relationships: is a type of transferase activity [GO:0016740] Also known as: transferase activity, transferring selenium-containing groups Sources: GOC:jl, ISBN:0198506732 Definition: Catalysis of the transfer of a selenium-containing group from one compound (donor) to another (acceptor). Subtypes: L-seryl-tRNA(Sec) selenium transferase activity [GO:0004125], GO:0043828, O-phosphoseryl-tRNA(Sec) selenium transferase activity [GO:0098621]